{
  "gene_name": "Phospholipid-transporting ATPase ID",
  "gene": "UniProtKB:P98198",
  "term_label": "trans-Golgi network",
  "gene_symbol": "ATP8B2",
  "term_id": "GO:0005802"
}